negative regulation of (Z)-nonadeca-1,14-diene biosynthetic process [GO:1900942] (biological process) Definition: Any process that stops, prevents or reduces the frequency, rate or extent of (Z)-nonadeca-1,14-diene biosynthetic process. Relationships: is a type of GO:1900912; is a type of regulation of (Z)-nonadeca-1,14-diene biosynthetic process [GO:1900941]; negatively regulates (Z)-nonadeca-1,14-diene biosynthetic process [GO:1900879] Sources: GOC:TermGenie, GOC:mengo_curators Also known as: down regulation of (Z)-nonadeca-1,14-diene anabolism, down regulation of (Z)-nonadeca-1,14-diene biosynthesis, down regulation of (Z)-nonadeca-1,14-diene biosynthetic process, down regulation of (Z)-nonadeca-1,14-diene formation, down regulation of (Z)-nonadeca-1,14-diene synthesis, down-regulation of (Z)-nonadeca-1,14-diene anabolism, down-regulation of (Z)-nonadeca-1,14-diene biosynthesis, down-regulation of (Z)-nonadeca-1,14-diene biosynthetic process, down-regulation of (Z)-nonadeca-1,14-diene formation, down-regulation of (Z)-nonadeca-1,14-diene synthesis, downregulation of (Z)-nonadeca-1,14-diene anabolism, downregulation of (Z)-nonadeca-1,14-diene biosynthesis, downregulation of (Z)-nonadeca-1,14-diene biosynthetic process, downregulation of (Z)-nonadeca-1,14-diene formation, downregulation of (Z)-nonadeca-1,14-diene synthesis, negative regulation of (Z)-nonadeca-1,14-diene anabolism, negative regulation of (Z)-nonadeca-1,14-diene biosynthesis, negative regulation of (Z)-nonadeca-1,14-diene formation, negative regulation of (Z)-nonadeca-1,14-diene synthesis, inhibition of (Z)-nonadeca-1,14-diene anabolism, inhibition of (Z)-nonadeca-1,14-diene biosynthesis, inhibition of (Z)-nonadeca-1,14-diene biosynthetic process, inhibition of (Z)-nonadeca-1,14-diene formation, inhibition of (Z)-nonadeca-1,14-diene synthesis